{
  "gene": "UniProtKB:Q5H8A3",
  "term_label": "Unknown biological process",
  "gene_symbol": "NMS",
  "gene_name": "Neuromedin-S",
  "term_id": "UNKNOWN:0002"
}